{
  "gene_symbol": "OR10J6P",
  "gene_name": "Putative olfactory receptor 10J6",
  "term_id": "GO:0004984",
  "term_label": "olfactory receptor activity",
  "gene": "UniProtKB:Q8NGY7"
}